{
  "gene_symbol": "YJU2",
  "gene": "UniProtKB:Q9BW85",
  "term_label": "first spliceosomal transesterification activity",
  "gene_name": "Splicing factor YJU2",
  "term_id": "GO:0000384"
}